{
  "gene": "UniProtKB:O95750",
  "term_id": "GO:0008543",
  "gene_symbol": "FGF19",
  "gene_name": "Fibroblast growth factor 19",
  "term_label": "fibroblast growth factor receptor signaling pathway"
}